{
  "gene_symbol": "RBCK1",
  "gene_name": "RanBP-type and C3HC4-type zinc finger-containing protein 1",
  "term_id": "GO:0043123",
  "gene": "UniProtKB:Q9BYM8",
  "term_label": "positive regulation of canonical NF-kappaB signal transduction"
}